{
  "gene_name": "Putative uncharacterized protein BVES-AS1",
  "gene": "UniProtKB:Q5T3Y7",
  "gene_symbol": "BVES-AS1",
  "term_id": "UNKNOWN:0001",
  "term_label": "Unknown molecular function"
}